{
  "term_label": "UDP-N-acetylglucosamine transmembrane transporter activity",
  "term_id": "GO:0005462",
  "gene": "UniProtKB:Q969S0",
  "gene_symbol": "SLC35B4",
  "gene_name": "Nucleotide sugar transporter SLC35B4"
}